dimethylargininase activity [GO:0016403] (molecular function) Definition: Catalysis of the reaction: N(G),N(G)-dimethyl-L-arginine + H2O = dimethylamine + L-citrulline. Also known as: N(G),N(G)-dimethylarginine dimethylaminohydrolase activity, NG,NG-dimethyl-L-arginine dimethylamidohydrolase activity, NG,NG-dimethylarginine dimethylaminohydrolase activity, dimethylarginine dimethylaminohydrolase activity Relationships: is a type of hydrolase activity, acting on carbon-nitrogen (but not peptide) bonds, in linear amidines [GO:0016813] Sources: EC:3.5.3.18